{
  "gene_symbol": "MLX",
  "gene": "UniProtKB:Q9UH92",
  "term_id": "GO:0005634",
  "gene_name": "Max-like protein X",
  "term_label": "nucleus"
}